{
  "gene_symbol": "DOCK11",
  "gene": "UniProtKB:Q5JSL3",
  "gene_name": "Dedicator of cytokinesis protein 11",
  "term_id": "GO:0035023",
  "term_label": "regulation of Rho protein signal transduction"
}